{
  "term_label": "protein ubiquitination",
  "gene_symbol": "DTX3L",
  "gene": "UniProtKB:Q8TDB6",
  "gene_name": "E3 ubiquitin-protein ligase DTX3L",
  "term_id": "GO:0016567"
}